exonucleolytic trimming to generate mature 5'-end of 5.8S rRNA from tricistronic rRNA transcript (SSU-rRNA, 5.8S rRNA, LSU-rRNA) [GO:0000465] (biological process) References: PMID:10690410 Sources: GOC:krc Relationships: is a type of GO:0000967; is part of maturation of 5.8S rRNA from tricistronic rRNA transcript (SSU-rRNA, 5.8S rRNA, LSU-rRNA) [GO:0000466] Definition: Exonucleolytic digestion of a pre-rRNA molecule to generate the mature 5'-end of a 5.8S rRNA molecule derived from an originally tricistronic pre-rRNA transcript that contained the Small Subunit (SSU) rRNA, the 5.8S rRNA, and the Large Subunit (LSU) rRNA in that order from 5' to 3' along the primary transcript.